{
  "term_label": "neuron migration",
  "gene_symbol": "DCC",
  "gene_name": "Netrin receptor DCC",
  "gene": "UniProtKB:P43146",
  "term_id": "GO:0001764"
}